{
  "gene": "UniProtKB:Q8IWS0",
  "gene_name": "PHD finger protein 6",
  "gene_symbol": "PHF6",
  "term_id": "GO:0005634",
  "term_label": "nucleus"
}